{
  "gene_name": "CNK3_IPCEF1 fusion protein",
  "term_label": "Unknown cellular component",
  "gene": "UniProtKB:G9CGD6",
  "gene_symbol": "CNK3/IPCEF1",
  "term_id": "UNKNOWN:0003"
}